{
  "gene": "UniProtKB:Q8NHS0",
  "gene_symbol": "DNAJB8",
  "gene_name": "DnaJ homolog subfamily B member 8",
  "term_id": "GO:0051082",
  "term_label": "unfolded protein binding"
}